{
  "term_label": "mitophagy",
  "term_id": "GO:0000423",
  "gene_name": "Beclin-2",
  "gene": "UniProtKB:A8MW95",
  "gene_symbol": "BECN2"
}